{
  "term_label": "nucleus",
  "gene": "UniProtKB:Q6ZMN8",
  "gene_symbol": "CCNI2",
  "term_id": "GO:0005634",
  "gene_name": "Cyclin-I2"
}